interleukin-9 receptor binding [GO:0005140] (molecular function) Definition: Binding to an interleukin-9 receptor. Sources: GOC:ai Also known as: IL-9, interleukin-9 receptor ligand Relationships: is a type of cytokine receptor binding [GO:0005126]; is a type of growth factor receptor binding [GO:0070851]